embryonic heart tube anterior/posterior pattern specification [GO:0035054] (biological process) Definition: The establishment, maintenance and elaboration of cell differentiation that results in the anterior/posterior subdivision of the embryonic heart tube. In Drosophila this results in subdivision of the dorsal vessel into to the posterior heart proper and the anterior aorta. References: PMID:12435360 Sources: GOC:bf Relationships: is a type of anterior/posterior pattern specification [GO:0009952]; is part of heart development [GO:0007507]